{
  "term_label": "cell adhesion mediated by integrin",
  "gene": "UniProtKB:P18564",
  "gene_symbol": "ITGB6",
  "term_id": "GO:0033627",
  "gene_name": "Integrin beta-6"
}